{
  "gene_symbol": "KRIT1",
  "term_id": "GO:2000114",
  "term_label": "regulation of establishment of cell polarity",
  "gene": "UniProtKB:O00522",
  "gene_name": "Krev interaction trapped protein 1"
}